{
  "gene": "UniProtKB:Q8NGU4",
  "term_id": "GO:0005886",
  "term_label": "plasma membrane",
  "gene_symbol": "OR2I1",
  "gene_name": "Putative olfactory receptor 2I1"
}